{
  "gene_name": "Transcription factor AP-2-beta",
  "gene_symbol": "TFAP2B",
  "term_label": "RNA polymerase II transcription regulatory region sequence-specific DNA binding",
  "gene": "UniProtKB:Q92481",
  "term_id": "GO:0000977"
}